{
  "gene_symbol": "GSTT2",
  "term_label": "glutathione metabolic process",
  "gene": "UniProtKB:P0CG29",
  "term_id": "GO:0006749",
  "gene_name": "Glutathione S-transferase theta-2"
}